regulation of sexual sporulation [GO:0034306] (biological process) Definition: Any process that modulates the frequency, rate or extent of spore formation from the products of meiosis. An example of this is found in Saccharomyces cerevisiae. Sources: GOC:mah Also known as: regulation of meiotic spore formation, regulation of meiotic sporulation, regulation of sexual spore formation, MAPKKK cascade during sporulation Relationships: is a type of regulation of sporulation [GO:0043937]; is a type of GO:0051445; regulates GO:0034293 Subtypes: regulation of sexual sporulation resulting in formation of a cellular spore [GO:0043940]